{
  "gene_name": "B-cell lymphoma_leukemia 10",
  "term_label": "transcription coactivator activity",
  "gene": "UniProtKB:O95999",
  "gene_symbol": "BCL10",
  "term_id": "GO:0003713"
}